{
  "gene_name": "Phosphatidylinositol 3,4,5-trisphosphate 5-phosphatase 2",
  "term_id": "GO:0043569",
  "gene_symbol": "INPPL1",
  "term_label": "negative regulation of insulin-like growth factor receptor signaling pathway",
  "gene": "UniProtKB:O15357"
}